{
  "term_label": "galactosylceramidase activity",
  "term_id": "GO:0004336",
  "gene_name": "Galactocerebrosidase",
  "gene_symbol": "GALC",
  "gene": "UniProtKB:P54803"
}